{
  "gene_name": "Uncharacterized protein C8orf90",
  "gene_symbol": "C8orf90",
  "term_id": "UNKNOWN:0002",
  "gene": "UniProtKB:A0A2R8Y2Y2",
  "term_label": "Unknown biological process"
}